{
  "term_label": "external side of plasma membrane",
  "gene_symbol": "IL2RB",
  "term_id": "GO:0009897",
  "gene_name": "Interleukin-2 receptor subunit beta",
  "gene": "UniProtKB:P14784"
}